{
  "gene": "UniProtKB:Q8NFU1",
  "term_label": "chloride transmembrane transport",
  "gene_name": "Bestrophin-2",
  "term_id": "GO:1902476",
  "gene_symbol": "BEST2"
}